{
  "gene": "UniProtKB:P41743",
  "gene_name": "Protein kinase C iota type",
  "term_label": "cellular response to insulin stimulus",
  "term_id": "GO:0032869",
  "gene_symbol": "PRKCI"
}